{
  "gene_symbol": "MAMLD1",
  "gene_name": "Mastermind-like domain-containing protein 1",
  "term_label": "Unknown molecular function",
  "term_id": "UNKNOWN:0001",
  "gene": "UniProtKB:Q13495"
}